{
  "gene_symbol": "NRXN1",
  "term_label": "trans-synaptic protein complex",
  "gene_name": "Neurexin-1",
  "gene": "UniProtKB:Q9ULB1",
  "term_id": "GO:0098820"
}